{
  "gene_symbol": "POMGNT2",
  "term_label": "protein O-linked glycosylation via mannose",
  "gene": "UniProtKB:Q8NAT1",
  "gene_name": "Protein O-linked-mannose beta-1,4-N-acetylglucosaminyltransferase 2",
  "term_id": "GO:0035269"
}